{
  "gene_symbol": "C7",
  "term_label": "Unknown molecular function",
  "gene": "UniProtKB:P10643",
  "term_id": "UNKNOWN:0001",
  "gene_name": "Complement component C7"
}